{
  "gene": "UniProtKB:P50213",
  "gene_symbol": "IDH3A",
  "gene_name": "Isocitrate dehydrogenase [NAD] subunit alpha, mitochondrial",
  "term_label": "mitochondrion",
  "term_id": "GO:0005739"
}